{
  "gene_name": "(Lyso)-N-acylphosphatidylethanolamine lipase",
  "term_label": "lipid droplet",
  "term_id": "GO:0005811",
  "gene": "UniProtKB:Q8TB40",
  "gene_symbol": "ABHD4"
}